{
  "gene_name": "ARL14 effector protein-like",
  "gene_symbol": "ARL14EPL",
  "term_id": "UNKNOWN:0002",
  "term_label": "Unknown biological process",
  "gene": "UniProtKB:P0DKL9"
}